{
  "term_id": "GO:0006357",
  "gene": "UniProtKB:O60479",
  "term_label": "regulation of transcription by RNA polymerase II",
  "gene_name": "Homeobox protein DLX-3",
  "gene_symbol": "DLX3"
}